columnar/cuboidal epithelial cell development [GO:0002066] (biological process) Sources: GOC:dph Subtypes: glandular epithelial cell development [GO:0002068], pancreatic D cell development [GO:0003324], intestinal epithelial cell development [GO:0060576] Definition: The process whose specific outcome is the progression of a columnar/cuboidal epithelial cell over time, from its formation to the mature structure. A columnar/cuboidal epithelial cell is a cell usually found in a two dimensional sheet with a free surface. Columnar/cuboidal epithelial cells take on the shape of a column or cube. Relationships: is a type of epithelial cell development [GO:0002064]; is part of GO:0002065